{
  "term_label": "interstrand cross-link repair",
  "gene": "UniProtKB:Q9H816",
  "gene_name": "5' exonuclease Apollo",
  "term_id": "GO:0036297",
  "gene_symbol": "DCLRE1B"
}